positive regulation of gastro-intestinal system smooth muscle contraction [GO:1904306] (biological process) Definition: Any process that activates or increases the frequency, rate or extent of gastro-intestinal system smooth muscle contraction. Relationships: is a type of GO:0045987; is a type of regulation of gastro-intestinal system smooth muscle contraction [GO:1904304]; positively regulates gastro-intestinal system smooth muscle contraction [GO:0014831] Also known as: up regulation of gastro-intestinal system smooth muscle contraction, up-regulation of gastro-intestinal system smooth muscle contraction, upregulation of gastro-intestinal system smooth muscle contraction, activation of gastro-intestinal system smooth muscle contraction References: PMID:10821044 Sources: GOC:TermGenie, GO_REF:0000058 Subtypes: positive regulation of stomach fundus smooth muscle contraction [GO:0120069], positive regulation of pyloric antrum smooth muscle contraction [GO:0120072], positive regulation of colon smooth muscle contraction [GO:1904343], GO:1904349